{
  "term_id": "GO:0006346",
  "gene_symbol": "MBD3L5",
  "gene": "UniProtKB:A6NJ08",
  "gene_name": "Putative methyl-CpG-binding domain protein 3-like 5",
  "term_label": "DNA methylation-dependent constitutive heterochromatin formation"
}